regulation of glutamatergic neuron differentiation [GO:0120006] (biological process) Definition: Any process that modulates the frequency, rate or extent of glutamatergic neuron differentiation. Relationships: is a type of regulation of neuron differentiation [GO:0045664]; RO_0002211 glutamatergic neuron differentiation [GO:1905962] Subtypes: negative regulation of glutamatergic neuron differentiation [GO:0120007], GO:0120008 References: PMID:24030726